{
  "term_label": "Unknown cellular component",
  "gene_name": "Heart- and neural crest derivatives-expressed protein 1",
  "term_id": "UNKNOWN:0003",
  "gene_symbol": "HAND1",
  "gene": "UniProtKB:O96004"
}